{
  "gene_name": "Protein monoglycylase TTLL8",
  "gene_symbol": "TTLL8",
  "term_id": "GO:0070736",
  "term_label": "protein-glycine ligase activity, initiating",
  "gene": "UniProtKB:A6PVC2"
}